spermatogenesis [GO:0007283] (biological process) Definition: The developmental process by which male germ line stem cells self renew or give rise to successive cell types resulting in the development of a spermatozoa. References: PMID:28073824, PMID:30990821 Sources: GOC:jid, ISBN:9780878933846 Also known as: generation of spermatozoa Relationships: is a type of developmental process involved in reproduction [GO:0003006]; is a type of male gamete generation [GO:0048232]